phosphatidylinositol 3-kinase inhibitor activity [GO:0141039] (molecular function) Definition: Binds to and decreases the activity of a phosphatidylinositol 3-kinase (PI3K). References: PMID:31686003 Relationships: is_a GO:0035014